{
  "gene": "UniProtKB:Q8N142",
  "gene_name": "Adenylosuccinate synthetase isozyme 1",
  "gene_symbol": "ADSS1",
  "term_label": "IMP metabolic process",
  "term_id": "GO:0046040"
}